{
  "gene_name": "ATPase family gene 2 protein homolog B",
  "term_id": "GO:0034098",
  "gene": "UniProtKB:Q9BVQ7",
  "gene_symbol": "AFG2B",
  "term_label": "VCP-NPL4-UFD1 AAA ATPase complex"
}